protein geranylgeranyltransferase activity [GO:0004661] (MF) Subtypes: CAAX-protein geranylgeranyltransferase activity [GO:0004662], Rab geranylgeranyltransferase activity [GO:0004663], geranylgeranyltransferase type III activity [GO:0170068] References: PMID:8621375 Definition: Catalysis of the covalent addition of a geranylgeranyl (20-carbon isoprenoid) group via thioether linkages to a cysteine residue at or near the C terminus of a protein. Relationships: is a type of GO:0008318 Also known as: protein-cysteine geranylgeranyltransferase activity